{
  "gene_symbol": "SYNM",
  "term_label": "structural constituent of muscle",
  "term_id": "GO:0008307",
  "gene": "UniProtKB:O15061",
  "gene_name": "Synemin"
}